adenohypophysis morphogenesis [GO:0048855] (biological process) Sources: GOC:cvs, GOC:dgh, GOC:dph, GOC:jid Definition: The process in which the anatomical structures of the adenohypophysis are generated and organized. The adenohypophysis is the anterior part of the pituitary. It secretes a variety of hormones and its function is regulated by the hypothalamus. Also known as: adenophysis morphogenesis, anterior pituitary gland morphogenesis, anterior pituitary morphogenesis Relationships: is a type of anatomical structure morphogenesis [GO:0009653]; is part of GO:0021984; is part of hypophysis morphogenesis [GO:0048850]